{
  "gene_name": "Unconventional myosin-VI",
  "gene": "UniProtKB:Q9UM54",
  "gene_symbol": "MYO6",
  "term_label": "actin cytoskeleton",
  "term_id": "GO:0015629"
}